{
  "gene_name": "Zinc finger protein 354B",
  "term_label": "regulation of transcription by RNA polymerase II",
  "gene": "UniProtKB:Q96LW1",
  "gene_symbol": "ZNF354B",
  "term_id": "GO:0006357"
}